{
  "term_label": "ATPase-coupled transmembrane transporter activity",
  "gene_name": "ATP-binding cassette sub-family A member 2",
  "gene_symbol": "ABCA2",
  "gene": "UniProtKB:Q9BZC7",
  "term_id": "GO:0042626"
}